{
  "gene": "UniProtKB:Q86SG7",
  "term_id": "GO:0005576",
  "gene_symbol": "LYG2",
  "gene_name": "Lysozyme g-like protein 2",
  "term_label": "extracellular region"
}